BAT3 complex binding [GO:1904288] (MF) References: PMID:23246001 Sources: GOC:PARL, GOC:TermGenie, GOC:bf Relationships: is a type of GO:0044877 Also known as: BAG6-UBL4A-TRC35 complex binding, Bag6 complex binding, BAT3-TRC35-UBL4A complex binding Definition: Binding to a BAT3 complex.